{
  "gene": "UniProtKB:O75689",
  "gene_symbol": "ADAP1",
  "term_id": "GO:0005547",
  "gene_name": "Arf-GAP with dual PH domain-containing protein 1",
  "term_label": "phosphatidylinositol-3,4,5-trisphosphate binding"
}